{
  "gene_name": "Plasma membrane calcium-transporting ATPase 2",
  "gene_symbol": "ATP2B2",
  "term_id": "GO:0005886",
  "term_label": "plasma membrane",
  "gene": "UniProtKB:Q01814"
}